{
  "term_id": "GO:0045944",
  "gene_name": "Methylcytosine dioxygenase TET1",
  "term_label": "positive regulation of transcription by RNA polymerase II",
  "gene_symbol": "TET1",
  "gene": "UniProtKB:Q8NFU7"
}